{
  "term_label": "DNA-binding transcription factor activity, RNA polymerase II-specific",
  "gene": "UniProtKB:P52740",
  "gene_symbol": "ZNF132",
  "term_id": "GO:0000981",
  "gene_name": "Zinc finger protein 132"
}